{
  "gene_symbol": "NSMCE1",
  "term_label": "nucleus",
  "gene_name": "Non-structural maintenance of chromosomes element 1 homolog",
  "term_id": "GO:0005634",
  "gene": "UniProtKB:Q8WV22"
}